{
  "gene_name": "Tubby-related protein 2",
  "gene": "UniProtKB:O00295",
  "term_id": "GO:0061512",
  "gene_symbol": "TULP2",
  "term_label": "protein localization to cilium"
}